positive regulation of seed germination [GO:0010030] (BP) Relationships: is a type of GO:0010029; is a type of GO:0048582; positively regulates seed germination [GO:0009845] Definition: Any process that activates or increase the rate of seed germination. Sources: GOC:sm Also known as: up regulation of seed germination, up-regulation of seed germination, upregulation of seed germination, activation of seed germination, stimulation of seed germination